{
  "term_id": "GO:0045180",
  "term_label": "basal cortex",
  "gene": "UniProtKB:Q86UU1",
  "gene_symbol": "PHLDB1",
  "gene_name": "Pleckstrin homology-like domain family B member 1"
}